{
  "term_id": "GO:0005911",
  "gene_name": "FERM domain-containing protein 1",
  "gene": "UniProtKB:Q8N878",
  "gene_symbol": "FRMD1",
  "term_label": "cell-cell junction"
}